{
  "term_label": "cytoplasm",
  "term_id": "GO:0005737",
  "gene_name": "Serine_threonine-protein kinase PAK 6",
  "gene_symbol": "PAK6",
  "gene": "UniProtKB:Q9NQU5"
}